NAD(P)H dehydrogenase complex (plastoquinone) [GO:0010598] (cellular component) Subtypes: NADH dehydrogenase complex (plastoquinone) [GO:0071685] Relationships: is a type of catalytic complex [GO:1902494] References: PMID:15608332 Definition: Complex that possesses NAD(P)H dehydrogenase (plastoquinone) activity. The complex is one of the components of the electron transport chain. It is involved in electron transport from an unidentified electron donor, possibly NADH, NADPH or ferredoxin(Fd) to the plastoquinone pool.